{
  "term_label": "transcription factor TFIID complex",
  "gene": "UniProtKB:Q5H9L4",
  "gene_name": "Transcription initiation factor TFIID subunit 7-like",
  "term_id": "GO:0005669",
  "gene_symbol": "TAF7L"
}